{
  "gene": "UniProtKB:P59780",
  "term_id": "UNKNOWN:0001",
  "gene_name": "AP-3 complex subunit sigma-2",
  "term_label": "Unknown molecular function",
  "gene_symbol": "AP3S2"
}